DNA clamp loader activity [GO:0003689] (molecular function) Relationships: is a type of GO:0008094; has part GO:0003677 References: PMID:16082778 Sources: GOC:mah, GOC:vw Also known as: DNA clamp loading ATPase activity, PCNA loading activity, PCNA loading complex activity, DNA-protein loading ATPase activity, protein-DNA loading ATPase activity Definition: Facilitating the opening of the ring structure of the PCNA complex, or any of the related sliding clamp complexes, and their closing around the DNA duplex, driven by ATP hydrolysis.